mammary gland fat development [GO:0060611] (BP) Definition: The progression of the mammary gland fat over time, from its formation to the mature structure. The mammary fat is an adipose structure in the gland that is invaded by the mammary ducts. Relationships: is_a adipose tissue development [GO:0060612]; is part of mammary gland development [GO:0030879] Sources: GOC:dph